{
  "gene": "UniProtKB:Q6UWM7",
  "term_id": "UNKNOWN:0001",
  "term_label": "Unknown molecular function",
  "gene_symbol": "LCTL",
  "gene_name": "Lactase-like protein"
}